porphyrin-containing compound metabolic process [GO:0006778] (biological process) Also known as: porphyrin metabolic process, porphyrin metabolism Subtypes: porphyrin-containing compound biosynthetic process [GO:0006779], porphyrin-containing compound catabolic process [GO:0006787], chlorophyll metabolic process [GO:0015994], GO:0042168, GO:0046501, GO:0046502 Sources: GOC:jl, ISBN:0198506732, Wikipedia:Porphyrin#Natural_formation Relationships: is a type of GO:0033013 Definition: The chemical reactions and pathways involving any member of a large group of derivatives or analogs of porphyrin. Porphyrins consists of a ring of four pyrrole nuclei linked each to the next at their alpha positions through a methine group.